eye pigmentation [GO:0048069] (biological process) Definition: Establishment of a pattern of pigment in the eye of an organism. Sources: GOC:jid Relationships: is a type of developmental pigmentation [GO:0048066] Subtypes: compound eye pigmentation [GO:0048072] Regulation: regulated by regulation of eye pigmentation [GO:0048073]; negatively regulated by GO:0048074; RO_0002213 by GO:0048075